{
  "gene_symbol": "KL",
  "term_label": "fibroblast growth factor binding",
  "gene": "UniProtKB:Q9UEF7",
  "gene_name": "Klotho",
  "term_id": "GO:0017134"
}